regulation of calcium ion-dependent exocytosis [GO:0017158] (biological process) Sources: GOC:go_curators Subtypes: GO:0045955, GO:0045956, regulation of calcium ion-dependent exocytosis of neurotransmitter [GO:1903233], regulation of dense core granule exocytosis [GO:1905413], regulation of acrosomal vesicle exocytosis [GO:2000367] Definition: Any process that modulates the frequency, rate or extent of calcium ion-dependent exocytosis. Relationships: is_a regulation of regulated secretory pathway [GO:1903305]; regulates calcium-ion regulated exocytosis [GO:0017156]